{
  "term_label": "sialylation",
  "term_id": "GO:0097503",
  "gene": "UniProtKB:Q96JF0",
  "gene_symbol": "ST6GAL2",
  "gene_name": "Beta-galactoside alpha-2,6-sialyltransferase 2"
}